canonical Wnt signaling pathway involved in mesenchymal stem cell differentiation [GO:0044338] (biological process) Definition: The series of molecular signals initiated by binding of a Wnt protein to a frizzled family receptor on the surface of the target cell, followed by propagation of the signal via beta-catenin, and ending with a change in transcription of target genes involved in mesenchymal stem cell differentiation. Sources: GOC:BHF, GOC:jl Relationships: is a type of canonical Wnt signaling pathway [GO:0060070]; is part of mesenchymal stem cell differentiation [GO:0072497] Also known as: canonical Wnt receptor signaling pathway involved in mesenchymal stem cell differentiation, canonical Wnt receptor signalling pathway involved in mesenchymal stem cell differentiation, canonical Wnt-activated signaling pathway involved in mesenchymal stem cell differentiation